{
  "term_id": "GO:0006338",
  "gene_symbol": "KDM4B",
  "gene": "UniProtKB:O94953",
  "term_label": "chromatin remodeling",
  "gene_name": "Lysine-specific demethylase 4B"
}